{
  "term_id": "UNKNOWN:0002",
  "gene_symbol": "RIMOC1",
  "term_label": "Unknown biological process",
  "gene_name": "RAB7A-interacting MON1-CCZ1 complex subunit 1",
  "gene": "UniProtKB:A6NDU8"
}